{
  "gene": "UniProtKB:Q5VWI1",
  "gene_name": "Transcription elongation regulator 1-like protein",
  "term_label": "Unknown biological process",
  "term_id": "UNKNOWN:0002",
  "gene_symbol": "TCERG1L"
}